{
  "gene_name": "cAMP-specific 3',5'-cyclic phosphodiesterase 4B",
  "gene_symbol": "PDE4B",
  "gene": "UniProtKB:Q07343",
  "term_id": "UNKNOWN:0003",
  "term_label": "Unknown cellular component"
}